Grb2-SHP-2 complex [GO:0070720] (cellular component) Definition: A protein complex that contains the receptor adaptor proteins Grb2 and SHP-2, and is involved signaling via the PDGFR signaling pathway. References: PMID:8943348 Sources: GOC:mah Also known as: GRB2-SHP-2 complex, PDGF stimulated Relationships: is_a plasma membrane protein complex [GO:0098797]